{
  "term_label": "olfactory receptor activity",
  "term_id": "GO:0004984",
  "gene": "UniProtKB:Q6IFG1",
  "gene_name": "Olfactory receptor 52E8",
  "gene_symbol": "OR52E8"
}